{
  "term_id": "UNKNOWN:0002",
  "gene": "UniProtKB:Q8IXM7",
  "gene_name": "Outer dense fiber protein 3-like protein 1",
  "gene_symbol": "CIMAP1C",
  "term_label": "Unknown biological process"
}